{
  "gene_name": "HLA class I histocompatibility antigen, alpha chain G",
  "gene_symbol": "HLA-G",
  "term_label": "signaling receptor binding",
  "term_id": "GO:0005102",
  "gene": "UniProtKB:P17693"
}